positive regulation of the force of heart contraction by circulating epinephrine-norepinephrine [GO:0003089] (biological process) Sources: GOC:mtg_cardio Definition: Any process that increases the force with which the cardiac muscles of the heart pump blood through the circulatory system as a result of the presence of epinephrine or norepinephrine in the bloodstream. Also known as: increased force of heart contraction by circulating adrenaline-noradrenaline, increased force of heart contraction by circulating epinephrine-norepinephrine, increased force of heart contraction by epinephrine-norepinephrine in the blood stream, positive regulation of heart contraction by circulating adrenaline-noradrenaline, positive regulation of heart contraction by circulating epinephrine-norepinephrine Relationships: is a type of GO:0001997